{
  "gene": "UniProtKB:Q5VWZ2",
  "term_label": "cytoplasm",
  "term_id": "GO:0005737",
  "gene_symbol": "LYPLAL1",
  "gene_name": "Lysophospholipase-like protein 1"
}